symbiont-mediated activation of host signal transduction pathway [GO:0052028] (biological process) Subtypes: symbiont-mediated activation of host NF-kappaB cascade [GO:0085033], symbiont-mediated activation of host MAPK cascade [GO:0141071], symbiont-mediated activation of host inflammasome-mediated signal transduction [GO:0141079], GO:0141080, symbiont-mediated activation of host G protein-coupled receptor signal transduction [GO:0141104], symbiont-mediated activation of host signal transduction pathway via agonism of host cell surface receptor [GO:0141134], GO:0141184 Relationships: is a type of symbiont-mediated perturbation of host signal transduction pathway [GO:0052027] Definition: A process in which a symbiont subverts a signal transduction pathway in the host organism by initiating, promoting, or enhancing its activation. The host is defined as the larger of the organisms involved in a symbiotic interaction. Also known as: positive regulation by organism of signal transduction in other organism involved in symbiotic interaction, positive regulation of signal transduction in other organism, induction by symbiont of host signal transduction pathway, positive regulation by symbiont of host signal transduction pathway, up regulation by symbiont of host signal transduction pathway, up-regulation by symbiont of host signal transduction pathway, upregulation by symbiont of host signal transduction pathway, activation by symbiont of host signal transduction pathway, stimulation by symbiont of host signal transduction pathway Sources: GOC:mtg_pamgo_17jul06